{
  "term_id": "UNKNOWN:0001",
  "gene": "UniProtKB:Q502W6",
  "gene_symbol": "VWA3B",
  "term_label": "Unknown molecular function",
  "gene_name": "von Willebrand factor A domain-containing protein 3B"
}